angiotensin maturation [GO:0002003] (biological process) Definition: The process leading to the attainment of the full functional capacity of angiotensin by conversion of angiotensinogen into mature angiotensin in the blood. Also known as: angiotensin catabolic process in blood Relationships: is a type of peptide hormone processing [GO:0016486]; is part of regulation of angiotensin levels in blood [GO:0002002] Sources: ISBN:0721643949